{
  "gene_symbol": "NXF1",
  "term_id": "GO:0016973",
  "gene": "UniProtKB:Q9UBU9",
  "term_label": "poly(A)+ mRNA export from nucleus",
  "gene_name": "Nuclear RNA export factor 1"
}